{
  "gene_name": "Zinc finger protein 195",
  "term_id": "GO:0000981",
  "term_label": "DNA-binding transcription factor activity, RNA polymerase II-specific",
  "gene": "UniProtKB:O14628",
  "gene_symbol": "ZNF195"
}